{
  "term_id": "GO:0042273",
  "term_label": "ribosomal large subunit biogenesis",
  "gene_symbol": "MRTO4",
  "gene_name": "mRNA turnover protein 4 homolog",
  "gene": "UniProtKB:Q9UKD2"
}